{
  "term_id": "GO:0097208",
  "gene": "UniProtKB:P11686",
  "gene_symbol": "SFTPC",
  "gene_name": "Pulmonary surfactant-associated protein C",
  "term_label": "alveolar lamellar body"
}